{
  "gene": "UniProtKB:Q96RI8",
  "gene_symbol": "TAAR6",
  "term_label": "plasma membrane",
  "gene_name": "Trace amine-associated receptor 6",
  "term_id": "GO:0005886"
}